{
  "term_label": "extracellular space",
  "gene_symbol": "RAET1L",
  "gene_name": "UL16-binding protein 6",
  "term_id": "GO:0005615",
  "gene": "UniProtKB:Q5VY80"
}